{
  "gene_name": "Zinc finger protein 623",
  "term_id": "GO:0006357",
  "gene_symbol": "ZNF623",
  "term_label": "regulation of transcription by RNA polymerase II",
  "gene": "UniProtKB:O75123"
}